{
  "gene": "UniProtKB:P26374",
  "term_label": "vesicle-mediated transport",
  "term_id": "GO:0016192",
  "gene_name": "Rab proteins geranylgeranyltransferase component A 2",
  "gene_symbol": "CHML"
}